{
  "gene_symbol": "OR13H1",
  "term_id": "GO:0050911",
  "gene_name": "Olfactory receptor 13H1",
  "term_label": "detection of chemical stimulus involved in sensory perception of smell",
  "gene": "UniProtKB:Q8NG92"
}